{
  "gene_symbol": "CD6",
  "term_label": "scavenger receptor activity",
  "term_id": "GO:0005044",
  "gene": "UniProtKB:P30203",
  "gene_name": "T-cell differentiation antigen CD6"
}